{
  "gene_symbol": "UQCRQ",
  "term_label": "respiratory chain complex III",
  "gene": "UniProtKB:O14949",
  "term_id": "GO:0045275",
  "gene_name": "Cytochrome b-c1 complex subunit 8"
}